{
  "gene": "UniProtKB:Q96JB6",
  "term_id": "GO:0004720",
  "gene_name": "Lysyl oxidase homolog 4",
  "gene_symbol": "LOXL4",
  "term_label": "protein-lysine 6-oxidase activity"
}